{
  "gene_name": "Tubulin alpha-1A chain",
  "term_label": "GTP binding",
  "gene": "UniProtKB:Q71U36",
  "term_id": "GO:0005525",
  "gene_symbol": "TUBA1A"
}